{
  "gene_name": "Insulin-degrading enzyme",
  "term_label": "mitochondrion",
  "term_id": "GO:0005739",
  "gene": "UniProtKB:P14735",
  "gene_symbol": "IDE"
}